{
  "gene_name": "Homeobox protein MOX-2",
  "gene_symbol": "MEOX2",
  "term_id": "GO:0005634",
  "term_label": "nucleus",
  "gene": "UniProtKB:P50222"
}